{
  "term_label": "Unknown cellular component",
  "term_id": "UNKNOWN:0003",
  "gene": "UniProtKB:Q02548",
  "gene_name": "Paired box protein Pax-5",
  "gene_symbol": "PAX5"
}